regulation of B cell activation [GO:0050864] (biological process) Subtypes: regulation of B cell proliferation [GO:0030888], regulation of isotype switching [GO:0045191], regulation of B cell differentiation [GO:0045577], negative regulation of B cell activation [GO:0050869], GO:0050871 Also known as: regulation of B lymphocyte activation, regulation of B-cell activation, regulation of B-lymphocyte activation Relationships: is a type of regulation of lymphocyte activation [GO:0051249]; regulates B cell activation [GO:0042113] Sources: GOC:ai Definition: Any process that modulates the frequency, rate or extent of B cell activation.